{
  "gene_name": "Discoidin domain-containing receptor 2",
  "gene": "UniProtKB:Q16832",
  "term_id": "GO:0005886",
  "term_label": "plasma membrane",
  "gene_symbol": "DDR2"
}